{
  "gene_name": "Glutamate receptor ionotropic, kainate 4",
  "gene_symbol": "GRIK4",
  "term_label": "synaptic transmission, glutamatergic",
  "term_id": "GO:0035249",
  "gene": "UniProtKB:Q16099"
}